response to unfolded protein [GO:0006986] (biological process) Subtypes: detection of unfolded protein [GO:0002235], GO:0034620 Also known as: heat shock protein activity Note: Note that this term should not be confused with 'unfolded protein response ; GO:0030968', which refers to one specific response to the presence of unfolded proteins in the ER. Definition: Any process that results in a change in state or activity of a cell or an organism (in terms of movement, secretion, enzyme production, gene expression, etc.) as a result of an unfolded protein stimulus. Sources: GOC:jl Relationships: is a type of response to topologically incorrect protein [GO:0035966]